11-O-demethyl-17-O-deacetylvindoline O-methyltransferase activity [GO:0030766] (molecular function) Also known as: 11-demethyl-17-deacetylvindoline 11-methyltransferase activity, S-adenosyl-L-methionine:11-O-demethyl-17-O-deacetylvindoline 11-O-methyltransferase activity, S-adenosyl-L-methionine:16-hydroxytabersonine 16-O-methyltransferase activity, tabersonine 16-O-methyltransferase activity Sources: EC:2.1.1.94 Definition: Catalysis of the reaction: S-adenosyl-L-methionine + 11-O-demethyl-17-O-deacetylvindoline = S-adenosyl-L-homocysteine + 17-O-deacetylvindoline. Relationships: is a type of S-adenosylmethionine-dependent methyltransferase activity [GO:0008757]